{
  "gene_name": "T cell receptor beta joining 2-1",
  "gene": "UniProtKB:A0A0A0MTA7",
  "gene_symbol": "TRBJ2-1",
  "term_id": "UNKNOWN:0002",
  "term_label": "Unknown biological process"
}